mitotic DNA replication termination [GO:1902979] (biological process) Also known as: DNA replication termination involved in mitotic cell cycle DNA replication Relationships: is a type of nuclear DNA replication termination [GO:1902317]; is a type of mitotic cell cycle process [GO:1903047]; is part of mitotic DNA replication [GO:1902969] Definition: Any DNA replication termination involved in mitotic cell cycle DNA replication. Sources: GOC:TermGenie, GO_REF:0000060